{
  "term_id": "GO:0008284",
  "gene": "UniProtKB:P15018",
  "term_label": "positive regulation of cell population proliferation",
  "gene_name": "Leukemia inhibitory factor",
  "gene_symbol": "LIF"
}